{
  "term_id": "GO:0006893",
  "gene_name": "Exocyst complex component 8",
  "gene_symbol": "EXOC8",
  "gene": "UniProtKB:Q8IYI6",
  "term_label": "Golgi to plasma membrane transport"
}